{
  "gene_name": "HERV-H LTR-associating protein 1",
  "gene": "UniProtKB:C9JL84",
  "gene_symbol": "HHLA1",
  "term_label": "Unknown biological process",
  "term_id": "UNKNOWN:0002"
}